{
  "term_label": "mitotic spindle assembly checkpoint signaling",
  "gene_name": "Mitotic spindle assembly checkpoint protein MAD1",
  "gene_symbol": "MAD1L1",
  "gene": "UniProtKB:Q9Y6D9",
  "term_id": "GO:0007094"
}